{
  "gene_symbol": "PPIL2",
  "gene_name": "RING-type E3 ubiquitin-protein ligase PPIL2",
  "term_label": "catalytic step 2 spliceosome",
  "gene": "UniProtKB:Q13356",
  "term_id": "GO:0071013"
}